{
  "gene": "UniProtKB:Q96QH2",
  "gene_name": "PML-RARA-regulated adapter molecule 1",
  "gene_symbol": "PRAM1",
  "term_id": "UNKNOWN:0001",
  "term_label": "Unknown molecular function"
}